{
  "gene_name": "Uncharacterized protein C17orf78",
  "term_id": "UNKNOWN:0001",
  "term_label": "Unknown molecular function",
  "gene": "UniProtKB:Q8N4C9",
  "gene_symbol": "C17orf78"
}